sialylation [GO:0097503] (biological process) Subtypes: GO:1990743 Relationships: is a type of macromolecule modification [GO:0043412] Sources: GOC:cjm Definition: The covalent attachment of sialic acid to a substrate molecule.